{
  "gene_symbol": "RPL23",
  "gene": "UniProtKB:P62829",
  "gene_name": "Large ribosomal subunit protein uL14",
  "term_label": "Unknown biological process",
  "term_id": "UNKNOWN:0002"
}